{
  "term_label": "cholesterol transfer activity",
  "term_id": "GO:0120020",
  "gene": "UniProtKB:P06727",
  "gene_name": "Apolipoprotein A-IV",
  "gene_symbol": "APOA4"
}